positive regulation of embryonic pattern specification [GO:1902877] (biological process) Definition: Any process that activates or increases the frequency, rate or extent of embryonic pattern specification. Relationships: is a type of positive regulation of multicellular organismal process [GO:0051240]; is a type of GO:1902875; positively regulates embryonic pattern specification [GO:0009880] Also known as: up regulation of embryonic pattern specification, up-regulation of embryonic pattern specification, upregulation of embryonic pattern specification, activation of embryonic pattern specification, activation of ventral/lateral system, positive regulation of ventral/lateral system, up regulation of ventral/lateral system, up-regulation of ventral/lateral system, upregulation of ventral/lateral system References: PMID:16872597 Sources: GOC:TermGenie, GOC:mr, GO_REF:0000058